{
  "term_label": "dendrite",
  "gene": "UniProtKB:Q9P021",
  "gene_symbol": "CRIPT",
  "gene_name": "Cysteine-rich PDZ-binding protein",
  "term_id": "GO:0030425"
}